{
  "gene_symbol": "MAPK11",
  "gene": "UniProtKB:Q15759",
  "gene_name": "Mitogen-activated protein kinase 11",
  "term_label": "intracellular signal transduction",
  "term_id": "GO:0035556"
}